XMP salvage [GO:0032265] (biological process) Definition: Any process which produces xanthosine monophosphate from derivatives of it, without de novo synthesis. Sources: GOC:mah Relationships: is a type of XMP biosynthetic process [GO:0097293]; is a type of purine ribonucleotide salvage [GO:0106380]